{
  "gene_name": "ATPase family gene 2 protein homolog A",
  "term_id": "GO:0005737",
  "gene": "UniProtKB:Q8NB90",
  "term_label": "cytoplasm",
  "gene_symbol": "AFG2A"
}